{
  "term_label": "single-stranded DNA 3'-5' DNA exonuclease activity",
  "gene_name": "Meiosis-specific with OB domain-containing protein",
  "gene": "UniProtKB:Q8N635",
  "term_id": "GO:0008310",
  "gene_symbol": "MEIOB"
}